diffuse secondary thickening [GO:0080193] (biological process) Sources: GOC:dhl Definition: Lateral growth of the older parts of a stem that occurs when the central parenchyma cells and the not yet fully differentiated fiber cells of the bundle sheaths continue to undergo cell division and expansion for a long period of time, leading to an increase in girth of the stem. Relationships: is a type of lateral growth [GO:0080190] Note: Occurs in the stems (PO:0009047) of some Arecaceae (palms).